1,5-anhydro-D-fructose reductase (1,5-anhydro-D-mannitol-forming) activity [GO:0033712] (molecular function) Sources: EC:1.1.1.292, RHEA:24208 Also known as: 1,5-anhydro-D-mannitol:NADP+ oxidoreductase activity, AFR Relationships: is a type of oxidoreductase activity, acting on the CH-OH group of donors, NAD or NADP as acceptor [GO:0016616] Definition: Catalysis of the reaction: 1,5-anhydro-D-mannitol + NADP+ = 1,5-anhydro-D-fructose + H+ + NADPH.